{
  "gene_name": "Beta-tectorin",
  "gene": "UniProtKB:Q96PL2",
  "term_label": "cell surface",
  "term_id": "GO:0009986",
  "gene_symbol": "TECTB"
}